{
  "term_label": "toll-like receptor 4 signaling pathway",
  "term_id": "GO:0034142",
  "gene_name": "Lymphocyte antigen 96",
  "gene_symbol": "LY96",
  "gene": "UniProtKB:Q9Y6Y9"
}